{
  "gene_name": "Protein ABHD16B",
  "term_id": "UNKNOWN:0003",
  "gene": "UniProtKB:Q9H3Z7",
  "gene_symbol": "ABHD16B",
  "term_label": "Unknown cellular component"
}